{
  "term_id": "GO:0016020",
  "gene_name": "Mitochondrial potassium channel ATP-binding subunit",
  "gene_symbol": "ABCB8",
  "gene": "UniProtKB:Q9NUT2",
  "term_label": "membrane"
}